negative regulation of mast cell chemotaxis [GO:0060755] (biological process) Sources: GOC:dph, GOC:tb Relationships: is_a negative regulation of leukocyte chemotaxis [GO:0002689]; is a type of GO:0060753; negatively regulates GO:0002551 Definition: Any process that decreases the rate, frequency or extent of mast cell chemotaxis. Mast cell chemotaxis is the movement of a mast cell in response to an external stimulus.